{
  "gene": "UniProtKB:Q9ULD9",
  "term_id": "GO:0006357",
  "term_label": "regulation of transcription by RNA polymerase II",
  "gene_name": "Zinc finger protein 608",
  "gene_symbol": "ZNF608"
}